{
  "term_label": "Unknown cellular component",
  "gene_symbol": "CTRL",
  "gene_name": "Chymotrypsin-like protease CTRL-1",
  "term_id": "UNKNOWN:0003",
  "gene": "UniProtKB:P40313"
}